{
  "term_label": "Cul2-RING ubiquitin ligase complex",
  "gene_name": "Leucine-rich repeat-containing protein 75A",
  "term_id": "GO:0031462",
  "gene": "UniProtKB:Q8NAA5",
  "gene_symbol": "LRRC75A"
}